{
  "gene_name": "Zinc finger protein 134",
  "term_label": "RNA polymerase II cis-regulatory region sequence-specific DNA binding",
  "gene_symbol": "ZNF134",
  "term_id": "GO:0000978",
  "gene": "UniProtKB:P52741"
}